{
  "term_id": "GO:0004715",
  "gene": "UniProtKB:Q6J9G0",
  "gene_symbol": "STYK1",
  "gene_name": "Tyrosine-protein kinase STYK1",
  "term_label": "non-membrane spanning protein tyrosine kinase activity"
}